geranoyl-CoA carboxylase activity [GO:0047925] (molecular function) Definition: Catalysis of the reaction: ATP + bicarbonate + geranoyl-CoA = 3-(4-methylpent-3-en-1-yl)pent-2-enedioyl-CoA + ADP + 2 H+ + phosphate. Sources: EC:6.4.1.5, RHEA:17701 Also known as: geranoyl coenzyme A carboxylase activity, geranoyl-CoA:carbon-dioxide ligase (ADP-forming), geranyl-CoA carboxylase activity Relationships: is a type of GO:0016421